{
  "gene_name": "Mitochondrial amidoxime reducing component 2",
  "term_id": "UNKNOWN:0003",
  "gene": "UniProtKB:Q969Z3",
  "gene_symbol": "MTARC2",
  "term_label": "Unknown cellular component"
}